{
  "gene_symbol": "CDC5L",
  "term_id": "GO:0005681",
  "term_label": "spliceosomal complex",
  "gene_name": "Cell division cycle 5-like protein",
  "gene": "UniProtKB:Q99459"
}